{
  "gene_symbol": "USP12",
  "term_label": "cysteine-type deubiquitinase activity",
  "gene": "UniProtKB:O75317",
  "gene_name": "Ubiquitin carboxyl-terminal hydrolase 12",
  "term_id": "GO:0004843"
}